{
  "term_label": "oxidative phosphorylation",
  "gene": "UniProtKB:P14406",
  "gene_symbol": "COX7A2",
  "term_id": "GO:0006119",
  "gene_name": "Cytochrome c oxidase subunit 7A2, mitochondrial"
}